{
  "term_id": "GO:0033204",
  "gene": "UniProtKB:Q969H6",
  "term_label": "ribonuclease P RNA binding",
  "gene_name": "Ribonuclease P_MRP protein subunit POP5",
  "gene_symbol": "POP5"
}